{
  "term_label": "ubiquitin ligase complex",
  "gene_symbol": "RNF217",
  "term_id": "GO:0000151",
  "gene_name": "E3 ubiquitin-protein ligase RNF217",
  "gene": "UniProtKB:Q8TC41"
}